{
  "gene_name": "Glycosyltransferase-like domain-containing protein 1",
  "gene": "UniProtKB:Q4AE62",
  "gene_symbol": "GTDC1",
  "term_id": "GO:0016438",
  "term_label": "tRNA-queuosine(34) beta-mannosyltransferase activity"
}